{
  "gene_symbol": "FFAR1",
  "gene": "UniProtKB:O14842",
  "gene_name": "Free fatty acid receptor 1",
  "term_id": "GO:0032024",
  "term_label": "positive regulation of insulin secretion"
}